{
  "term_label": "Unknown molecular function",
  "gene_name": "T cell receptor delta variable 3",
  "term_id": "UNKNOWN:0001",
  "gene": "UniProtKB:A0JD37",
  "gene_symbol": "TRDV3"
}